{
  "term_id": "GO:0016020",
  "term_label": "membrane",
  "gene_name": "Acyl-CoA 6-desaturase",
  "gene_symbol": "FADS2",
  "gene": "UniProtKB:O95864"
}